{
  "term_id": "GO:0034354",
  "gene_name": "Indoleamine 2,3-dioxygenase 2",
  "gene": "UniProtKB:Q6ZQW0",
  "term_label": "'de novo' NAD+ biosynthetic process from L-tryptophan",
  "gene_symbol": "IDO2"
}